cell wall polysaccharide catabolic process [GO:0044347] (biological process) Relationships: is a type of GO:0000272; is a type of cell wall polysaccharide metabolic process [GO:0010383]; is a type of cell wall macromolecule catabolic process [GO:0016998] Sources: GOC:mengo_curators Definition: The chemical reactions and pathways resulting in the breakdown of cell wall polysaccharides. Subtypes: plant-type cell wall cellulose catabolic process [GO:0044348], mannan catabolic process [GO:0046355], GO:1902089, cell wall polysaccharide catabolic process involved in abscission [GO:1990076] Regulation: regulated by regulation of cell wall polysaccharide catabolic process [GO:2000966]; negatively regulated by negative regulation of cell wall polysaccharide catabolic process [GO:2000967]; positively regulated by positive regulation of cell wall polysaccharide catabolic process [GO:2000968] Also known as: cell wall polysaccharide breakdown